{
  "gene_name": "Myb-related protein B",
  "gene_symbol": "MYBL2",
  "gene": "UniProtKB:P10244",
  "term_label": "mitotic cell cycle",
  "term_id": "GO:0000278"
}